{
  "term_label": "Unknown cellular component",
  "gene": "UniProtKB:Q8N9W4",
  "gene_name": "Golgin subfamily A member 6-like protein 2",
  "term_id": "UNKNOWN:0003",
  "gene_symbol": "GOLGA6L2"
}